{
  "gene_name": "Toll-like receptor 6",
  "term_label": "cellular response to diacyl bacterial lipopeptide",
  "gene": "UniProtKB:Q9Y2C9",
  "gene_symbol": "TLR6",
  "term_id": "GO:0071726"
}